{
  "gene": "UniProtKB:Q5VTQ0",
  "gene_symbol": "TTC39B",
  "term_id": "UNKNOWN:0003",
  "term_label": "Unknown cellular component",
  "gene_name": "Tetratricopeptide repeat protein 39B"
}